{
  "gene": "UniProtKB:Q12772",
  "gene_symbol": "SREBF2",
  "gene_name": "Sterol regulatory element-binding protein 2",
  "term_label": "DNA-binding transcription factor activity, RNA polymerase II-specific",
  "term_id": "GO:0000981"
}